viral transcription [GO:0019083] (biological process) Sources: GOC:jl, ISBN:0781702534 Relationships: is a type of viral process [GO:0016032]; is part of viral gene expression [GO:0019080] Regulation: negatively regulated by negative regulation of viral transcription [GO:0032897]; regulated by regulation of viral transcription [GO:0046782]; positively regulated by positive regulation of viral transcription [GO:0050434] Definition: The process by which a viral genome, or part of a viral genome, is transcribed within the host cell. Subtypes: middle viral transcription [GO:0019084], early viral transcription [GO:0019085], late viral transcription [GO:0019086], GO:0039695, RNA-templated viral transcription [GO:0039696]